{
  "gene_symbol": "EGFR",
  "gene_name": "Epidermal growth factor receptor",
  "term_id": "GO:0007173",
  "term_label": "epidermal growth factor receptor signaling pathway",
  "gene": "UniProtKB:P00533"
}